{
  "term_label": "regulation of transcription by RNA polymerase II",
  "gene_symbol": "ZNF669",
  "gene_name": "Zinc finger protein 669",
  "term_id": "GO:0006357",
  "gene": "UniProtKB:Q96BR6"
}